{
  "gene": "UniProtKB:A6NIK2",
  "term_label": "Unknown cellular component",
  "gene_name": "Leucine-rich repeat-containing protein 10B",
  "gene_symbol": "LRRC10B",
  "term_id": "UNKNOWN:0003"
}